{
  "term_label": "cytosol",
  "gene_symbol": "AFG2B",
  "gene_name": "ATPase family gene 2 protein homolog B",
  "gene": "UniProtKB:Q9BVQ7",
  "term_id": "GO:0005829"
}